{
  "term_label": "RNA polymerase II cis-regulatory region sequence-specific DNA binding",
  "gene": "UniProtKB:Q68DI1",
  "gene_symbol": "ZNF776",
  "gene_name": "Zinc finger protein 776",
  "term_id": "GO:0000978"
}